{
  "gene": "UniProtKB:Q9Y2K7",
  "term_label": "transcription coregulator activity",
  "gene_symbol": "KDM2A",
  "term_id": "GO:0003712",
  "gene_name": "Lysine-specific demethylase 2A"
}